{
  "gene_name": "Coiled-coil domain-containing protein 40",
  "term_label": "cilium",
  "gene_symbol": "CCDC40",
  "gene": "UniProtKB:Q4G0X9",
  "term_id": "GO:0005929"
}